{
  "gene_symbol": "HK3",
  "gene_name": "Hexokinase-3",
  "term_id": "GO:0001678",
  "term_label": "intracellular glucose homeostasis",
  "gene": "UniProtKB:P52790"
}